negative regulation of ribosomal small subunit export from nucleus [GO:2000207] (biological process) Definition: Any process that stops, prevents, or reduces the frequency, rate or extent of ribosomal small subunit export from nucleus. Sources: GOC:mah Also known as: negative regulation of ribosomal small subunit export from cell nucleus, negative regulation of ribosomal small subunit export out of nucleus, negative regulation of ribosomal small subunit transport from nucleus to cytoplasm, negative regulation of ribosomal small subunit-nucleus export, negative regulation of 30S ribosomal subunit export from nucleus, negative regulation of 40S ribosomal subunit export from nucleus Relationships: is a type of negative regulation of ribosomal subunit export from nucleus [GO:2000201]; is a type of regulation of ribosomal small subunit export from nucleus [GO:2000206]; RO_0002212 ribosomal small subunit export from nucleus [GO:0000056]